{
  "gene_name": "Interleukin-1 receptor type 1",
  "gene_symbol": "IL1R1",
  "gene": "UniProtKB:P14778",
  "term_label": "interleukin-1 receptor activity",
  "term_id": "GO:0004908"
}